UUA codon-amino acid adaptor activity [GO:0033403] (molecular function) Definition: A triplet codon-amino acid adaptor activity that recognizes a UUA codon. Also known as: TTA codon-amino acid adaptor activity, leucine tRNA Sources: GOC:mah Relationships: is a type of triplet codon-amino acid adaptor activity [GO:0030533] Note: Note that in the standard genetic code, TTA codes for leucine.